{
  "gene": "UniProtKB:Q9Y3L3",
  "term_label": "regulation of actin cytoskeleton organization",
  "gene_symbol": "SH3BP1",
  "term_id": "GO:0032956",
  "gene_name": "SH3 domain-binding protein 1"
}